{
  "gene": "UniProtKB:Q9P2K6",
  "gene_name": "Kelch-like protein 42",
  "gene_symbol": "KLHL42",
  "term_label": "regulation of microtubule-based process",
  "term_id": "GO:0032886"
}